{
  "term_id": "UNKNOWN:0003",
  "gene_symbol": "CRB3",
  "gene": "UniProtKB:Q9BUF7",
  "term_label": "Unknown cellular component",
  "gene_name": "Protein crumbs homolog 3"
}